{
  "term_label": "cytokine receptor activity",
  "gene_symbol": "IFNGR2",
  "gene_name": "Interferon gamma receptor 2",
  "term_id": "GO:0004896",
  "gene": "UniProtKB:P38484"
}